{
  "term_id": "GO:0003924",
  "gene": "UniProtKB:P51159",
  "gene_symbol": "RAB27A",
  "gene_name": "Ras-related protein Rab-27A",
  "term_label": "GTPase activity"
}